sulfide:quinone oxidoreductase activity [GO:0070224] (molecular function) Definition: Catalysis of the reaction: H2S (hydrogen sulfide) + a quinone = S0 (sulfane sulfur) + a hydroquinone. Also known as: sulfide-quinone reductase activity, sulphide:quinone oxidoreductase activity Note: Note that EC:1.8.5.4 describes this reaction as bacterial-specific, but it has also been observed in eukaryotes (PMID:22852582, PMID:10224084). Sources: RHEA:30239 Relationships: is a type of oxidoreductase activity, acting on a sulfur group of donors, quinone or similar compound as acceptor [GO:0016672]